{
  "gene_name": "Cholecystokinin receptor type A",
  "term_id": "GO:0032870",
  "gene_symbol": "CCKAR",
  "term_label": "cellular response to hormone stimulus",
  "gene": "UniProtKB:P32238"
}